{
  "gene": "UniProtKB:P49754",
  "gene_symbol": "VPS41",
  "term_label": "vacuolar membrane",
  "term_id": "GO:0005774",
  "gene_name": "Vacuolar protein sorting-associated protein 41 homolog"
}